{
  "term_label": "Unknown cellular component",
  "gene_name": "Protein ABHD8",
  "term_id": "UNKNOWN:0003",
  "gene": "UniProtKB:Q96I13",
  "gene_symbol": "ABHD8"
}